{
  "term_label": "calcium ion export across plasma membrane",
  "gene": "UniProtKB:P32418",
  "term_id": "GO:1990034",
  "gene_symbol": "SLC8A1",
  "gene_name": "Sodium_calcium exchanger 1"
}